alpha-D-ribose 1-methylphosphonate 5-triphosphate synthase activity [GO:0061693] (molecular function) Definition: Catalysis of the reaction: ATP + methylphosphonate = alpha-D-ribose 1-methylphosphonate 5-triphosphate + adenine. Relationships: is a type of phosphotransferase activity, for other substituted phosphate groups [GO:0016780] References: PMID:22089136 Sources: EC:2.7.8.37, GOC:dph